{
  "gene": "UniProtKB:Q9UL58",
  "gene_name": "Zinc finger protein 215",
  "gene_symbol": "ZNF215",
  "term_label": "regulation of transcription by RNA polymerase II",
  "term_id": "GO:0006357"
}